{
  "term_label": "termination of mitochondrial transcription",
  "term_id": "GO:0006393",
  "gene": "UniProtKB:Q99551",
  "gene_symbol": "MTERF1",
  "gene_name": "Transcription termination factor 1, mitochondrial"
}